{
  "term_label": "smoothened signaling pathway",
  "gene_name": "Tectonic-3",
  "term_id": "GO:0007224",
  "gene": "UniProtKB:Q6NUS6",
  "gene_symbol": "TCTN3"
}